{
  "gene_symbol": "KITLG",
  "gene_name": "Kit ligand",
  "gene": "UniProtKB:P21583",
  "term_id": "GO:0005173",
  "term_label": "stem cell factor receptor binding"
}